anterior/posterior pattern specification [GO:0009952] (BP) Subtypes: somitogenesis [GO:0001756], anterior region determination [GO:0007355], thorax and anterior abdomen determination [GO:0007356], posterior abdomen determination [GO:0007359], GO:0007366, compartment pattern specification [GO:0007386], anterior/posterior pattern specification, imaginal disc [GO:0007448], spinal cord anterior/posterior patterning [GO:0021512], forebrain anterior/posterior pattern specification [GO:0021797], GO:0021903, neural plate anterior/posterior regionalization [GO:0021999], embryonic heart tube anterior/posterior pattern specification [GO:0035054], foregut regionalization [GO:0060423], anterior/posterior pattern specification involved in kidney development [GO:0072098] Also known as: anterior/posterior pattern formation Relationships: is_a regionalization [GO:0003002] Sources: GOC:dph, GOC:go_curators, GOC:isa_complete, GOC:tb Definition: The regionalization process in which specific areas of cell differentiation are determined along the anterior-posterior axis. The anterior-posterior axis is defined by a line that runs from the head or mouth of an organism to the tail or opposite end of the organism.